{
  "term_id": "UNKNOWN:0002",
  "gene_symbol": "CERCAM",
  "term_label": "Unknown biological process",
  "gene_name": "Inactive glycosyltransferase 25 family member 3",
  "gene": "UniProtKB:Q5T4B2"
}